G protein-coupled receptor activity [GO:0004930] (molecular function) Definition: Combining with an extracellular signal and transmitting the signal across the membrane by activating an associated G-protein; promotes the exchange of GDP for GTP on the alpha subunit of a heterotrimeric G-protein complex. Relationships: is_a transmembrane signaling receptor activity [GO:0004888]; is part of GO:0007186 Subtypes: G protein-coupled nucleotide receptor activity [GO:0001608], G protein-coupled adenosine receptor activity [GO:0001609], growth hormone secretagogue receptor activity [GO:0001616], pituitary adenylate cyclase-activating polypeptide receptor activity [GO:0001634], G protein-coupled chemoattractant receptor activity [GO:0001637], G protein-coupled cytokinin receptor activity [GO:0001647], cannabinoid receptor activity [GO:0004949], GO:0004953, GO:0004964, GO:0004965, gonadotropin-releasing hormone receptor activity [GO:0004968], G protein-coupled opioid receptor activity [GO:0004985], GO:0004991, GO:0004992, thyroid-stimulating hormone receptor activity [GO:0004996], thyrotropin-releasing hormone receptor activity [GO:0004997], vasoactive intestinal polypeptide receptor activity [GO:0004999], G protein-coupled photoreceptor activity [GO:0008020], G protein-coupled amine receptor activity [GO:0008227], melatonin receptor activity [GO:0008502], G protein-coupled peptide receptor activity [GO:0008528], secretin receptor activity [GO:0015055], corticotrophin-releasing factor receptor activity [GO:0015056], pheromone receptor activity [GO:0016503], gastric inhibitory peptide receptor activity [GO:0016519], growth hormone-releasing hormone receptor activity [GO:0016520], melanin-concentrating hormone receptor activity [GO:0030273], choriogonadotropin hormone receptor activity [GO:0035472], GO:0036505, GO:0038022, GO:0038054, G protein-coupled bile acid receptor activity [GO:0038182], GO:0042654, GO:0045028, GO:0045125, nicotinic acid receptor activity [GO:0070553], G protein-coupled pyrimidinergic nucleotide receptor activity [GO:0071553], GPCR taste receptor activity [GO:0090681], G protein-coupled glutamate receptor activity [GO:0098988], G protein-coupled neurotransmitter receptor activity [GO:0099528], GO:0099530, G protein-coupled folate receptor activity [GO:0106063], G protein-coupled chemorepellent receptor activity [GO:0140985], GO:1990576, mast cell secretagogue receptor activity [GO:1990595] Also known as: G protein coupled receptor activity, G protein linked receptor activity, G-protein coupled receptor activity, G-protein linked receptor activity, GPCR activity, ligand-dependent GPCR activity, receptor activity, G-protein coupled, EBV-induced receptor, Epstein-Barr Virus-induced receptor activity, G-protein coupled receptor activity, unknown ligand, Mas proto-oncogene receptor activity, RDC1 receptor activity, SREB receptor, orphan G protein coupled receptor activity, orphan G-protein coupled receptor activity, orphan GPCR activity, super conserved receptor expressed in brain receptor activity Sources: GOC:bf, Wikipedia:GPCR